{
  "term_id": "GO:0043330",
  "gene": "UniProtKB:P05015",
  "gene_symbol": "IFNA16",
  "term_label": "response to exogenous dsRNA",
  "gene_name": "Interferon alpha-16"
}